{
  "gene_name": "Lysine-rich coiled-coil protein 1",
  "term_label": "Unknown biological process",
  "gene_symbol": "KRCC1",
  "term_id": "UNKNOWN:0002",
  "gene": "UniProtKB:Q9NPI7"
}